{
  "gene": "UniProtKB:P60606",
  "term_id": "UNKNOWN:0001",
  "gene_symbol": "CTXN1",
  "gene_name": "Cortexin-1",
  "term_label": "Unknown molecular function"
}